nickel chaperone activity [GO:0170061] (molecular function) Definition: Directly binding to and delivering nickel ions to a target protein. References: PMID:32133383, PMID:34530332 Also known as: nickel carrier activity Relationships: is a type of metallochaperone activity [GO:0016530]